intermediate-density lipoprotein particle remodeling [GO:0034373] (BP) Relationships: is a type of triglyceride-rich lipoprotein particle remodeling [GO:0034370] Definition: The acquisition, loss or modification of a protein or lipid within an intermediate-density lipoprotein particle. Also known as: IDL remodeling, IDL remodelling, intermediate-density lipoprotein particle remodelling, intermediate-density lipoprotein particle formation Sources: GOC:BHF, GOC:expert_pt, GOC:mah, GOC:rl